{
  "term_label": "Unknown biological process",
  "gene_name": "Proline and serine-rich protein 1",
  "term_id": "UNKNOWN:0002",
  "gene_symbol": "PROSER1",
  "gene": "UniProtKB:Q86XN7"
}